{
  "term_label": "protein folding",
  "gene": "UniProtKB:Q6ZRP7",
  "term_id": "GO:0006457",
  "gene_symbol": "QSOX2",
  "gene_name": "Sulfhydryl oxidase 2"
}